D3 vitamins binding [GO:1902271] (molecular function) Definition: Binding to D3 vitamins. References: PMID:9127467 Sources: GOC:TermGenie, GOC:bf Relationships: is a type of vitamin D binding [GO:0005499] Subtypes: calcitriol binding [GO:1902098], calcidiol binding [GO:1902118]